{
  "gene": "UniProtKB:Q17RC7",
  "term_label": "SNARE binding",
  "gene_name": "Exocyst complex component 3-like protein 4",
  "term_id": "GO:0000149",
  "gene_symbol": "EXOC3L4"
}